{
  "term_id": "GO:0045277",
  "term_label": "respiratory chain complex IV",
  "gene": "UniProtKB:P24311",
  "gene_name": "Cytochrome c oxidase subunit 7B, mitochondrial",
  "gene_symbol": "COX7B"
}